choline monooxygenase (NADP+) activity [GO:0102280] (MF) Relationships: is_a choline dehydrogenase activity [GO:0008812] Also known as: choline monooxygenase activity (NADP-dependent) Definition: Catalysis of the reaction: choline + NADP+ = betaine aldehyde + NADPH + H+. References: PMID:21769646 Sources: GOC:pz